organometal metabolic process [GO:0018942] (biological process) References: PMID:36598231 Sources: ISBN:0198506732 Also known as: organometal metabolism Definition: The chemical reactions and pathways involving organometals, any metal-containing organic compound, especially one in which the metal atom is linked directly to one of more carbon atoms. Relationships: is a type of GO:0008152 Subtypes: tri-n-butyltin metabolic process [GO:0018944], GO:0019506, methylmercury biosynthetic process [GO:0042192], GO:0042193